{
  "term_label": "NSL complex",
  "gene_symbol": "KANSL1L",
  "term_id": "GO:0044545",
  "gene_name": "KAT8 regulatory NSL complex subunit 1-like protein",
  "gene": "UniProtKB:A0AUZ9"
}